{
  "gene": "UniProtKB:P57679",
  "term_label": "plasma membrane protein complex",
  "gene_name": "EvC complex member EVC",
  "term_id": "GO:0098797",
  "gene_symbol": "EVC"
}